protein-N(PI)-phosphohistidine-trehalose phosphotransferase system transporter activity [GO:0022879] (molecular function) Definition: Catalysis of the PEP-dependent, phosphoryl transfer-driven transport of substances across a membrane. The transport happens by catalysis of the reaction: protein N-phosphohistidine + trehalose(out) = protein histidine + trehalose phosphate(in). This differs from primary and secondary active transport in that the solute is modified during transport. Sources: GOC:mtg_transport, ISBN:0815340729 Relationships: is a type of protein-N(PI)-phosphohistidine-sugar phosphotransferase activity [GO:0008982]; is a type of GO:0015574 Also known as: trehalose PTS transporter activity